{
  "gene_symbol": "MYH7B",
  "gene": "UniProtKB:A7E2Y1",
  "term_label": "cytoplasm",
  "gene_name": "Myosin-7B",
  "term_id": "GO:0005737"
}